fungal-type cell wall (1->3)-alpha-glucan biosynthetic process [GO:0070600] (biological process) Also known as: fungal-type cell wall 1,3-alpha-glucan anabolism, fungal-type cell wall 1,3-alpha-glucan biosynthesis, fungal-type cell wall 1,3-alpha-glucan biosynthetic process, fungal-type cell wall 1,3-alpha-glucan formation, fungal-type cell wall 1,3-alpha-glucan synthesis, fungal-type cell wall alpha-1,3-glucan anabolism, fungal-type cell wall alpha-1,3-glucan biosynthesis, fungal-type cell wall alpha-1,3-glucan biosynthetic process, fungal-type cell wall alpha-1,3-glucan formation, fungal-type cell wall alpha-1,3-glucan synthesis Definition: The chemical reactions and pathways resulting in the formation of (1->3)-alpha-D-glucans, compounds composed of glucose residues linked by (1->3)-alpha-D-glucosidic bonds, found in fungal-type cell walls, including those of ascospores. Regulation: regulated by regulation of fungal-type cell wall (1->3)-alpha-glucan biosynthetic process [GO:0070610] Relationships: is a type of GO:0051278; is a type of cell wall (1->3)-alpha-glucan biosynthetic process [GO:0070598]; is a type of fungal-type cell wall (1->3)-alpha-glucan metabolic process [GO:0070599] Sources: GOC:mah